{
  "gene_name": "Structural maintenance of chromosomes protein 3",
  "gene": "UniProtKB:Q9UQE7",
  "term_label": "double-stranded DNA binding",
  "gene_symbol": "SMC3",
  "term_id": "GO:0003690"
}